{
  "gene_symbol": "PTTG1IP",
  "term_label": "protein import into nucleus",
  "gene": "UniProtKB:P53801",
  "gene_name": "Pituitary tumor-transforming gene 1 protein-interacting protein",
  "term_id": "GO:0006606"
}